synaptic vesicle transport [GO:0048489] (biological process) Definition: The directed movement of synaptic vesicles. Relationships: is a type of GO:0006810; is a type of GO:0009987; is a type of establishment of vesicle localization [GO:0051650]; is a type of synaptic vesicle localization [GO:0097479] Sources: GOC:aruk, GOC:bc, GOC:jid, GOC:lmg, GOC:pr Also known as: synaptic vesicle fission, synaptic vesicle fusion, synaptic vesicle trafficking Subtypes: synaptic vesicle cytoskeletal transport [GO:0099514] Regulation: regulated by GO:1902803; RO_0002212 by negative regulation of synaptic vesicle transport [GO:1902804]; positively regulated by positive regulation of synaptic vesicle transport [GO:1902805]